{
  "gene": "UniProtKB:Q7Z4V5",
  "term_id": "GO:0006338",
  "term_label": "chromatin remodeling",
  "gene_name": "Hepatoma-derived growth factor-related protein 2",
  "gene_symbol": "HDGFL2"
}